{
  "gene": "UniProtKB:Q96QE5",
  "gene_name": "Transcription elongation factor, mitochondrial",
  "term_id": "GO:0003711",
  "term_label": "transcription elongation factor activity",
  "gene_symbol": "TEFM"
}